{
  "gene": "UniProtKB:A5D8W1",
  "term_id": "GO:1902093",
  "term_label": "positive regulation of flagellated sperm motility",
  "gene_name": "Cilia- and flagella-associated protein 69",
  "gene_symbol": "CFAP69"
}